ribitol-5-phosphate 2-dehydrogenase [NAD(P)+] activity [GO:0050256] (molecular function) Definition: Catalysis of the reaction: D-ribitol 5-phosphate + NAD(P)+ = D-ribulose 5-phosphate + NAD(P)H + H+. Relationships: is_a oxidoreductase activity, acting on the CH-OH group of donors, NAD or NADP as acceptor [GO:0016616] Sources: EC:1.1.1.137 Also known as: D-ribitol-5-phosphate:NAD(P)+ 2-oxidoreductase activity, dehydrogenase, ribitol 5-phosphate